behavioral response to nicotine [GO:0035095] (biological process) Sources: GOC:bf, ISBN:0198506732 Also known as: behavioural response to nicotine Relationships: is a type of adult behavior [GO:0030534]; is part of response to nicotine [GO:0035094] Definition: Any process that results in a change in the behavior of an organism as a result of a nicotine stimulus.